positive regulation of striated muscle cell apoptotic process [GO:0010663] (BP) Also known as: positive regulation of striated muscle cell apoptosis Sources: GOC:dph, GOC:mtg_apoptosis, GOC:tb Relationships: is a type of positive regulation of muscle cell apoptotic process [GO:0010661]; is a type of GO:0010662; positively regulates striated muscle cell apoptotic process [GO:0010658] Definition: Any process that increases the rate or extent of striated muscle cell apoptotic process, a form of programmed cell death induced by external or internal signals that trigger the activity of proteolytic caspases whose actions dismantle a striated muscle cell and result in its death. Subtypes: positive regulation of cardiac muscle cell apoptotic process [GO:0010666]